macropinocytosis [GO:0044351] (biological process) Definition: An endocytosis process that results in the uptake of liquid material by cells from their external environment by the 'ruffling' of the cell membrane to form heterogeneously sized intracellular vesicles called macropinosomes, which can be up to 5 micrometers in size. Regulation: RO_0002211 by regulation of macropinocytosis [GO:1905301]; negatively regulated by GO:1905302; positively regulated by positive regulation of macropinocytosis [GO:1905303] Also known as: clathrin-independent pinocytosis, single-organism macropinocytosis Subtypes: extracellular exosome macropinocytosis [GO:0061707] Relationships: is a type of pinocytosis [GO:0006907] References: PMID:14732047